nuclear dicing body [GO:0010445] (cellular component) References: PMID:17442570 Also known as: D body Relationships: is a type of nuclear body [GO:0016604] Definition: A small round nuclear body, measuring 0.2-0.8 microns in diameter that is diffusely distributed throughout the nucleoplasm. Several proteins known to be involved in miRNA processing have been localized to these structures. D-bodies are thought to be involved in primary-miRNA processing and/or storage/assembly of miRNA processing complexes.